transport of virus in host, tissue to tissue [GO:0046741] (biological process) Relationships: is a type of transport of virus in multicellular host [GO:0046739] Also known as: spread of virus within host, tissue to tissue, tissue to tissue spread of virus within host, viral spread within host, tissue to tissue, spread of virus in host, tissue to tissue Sources: GOC:bf, GOC:jl, ISBN:0781718325 Definition: The transport of a virus between tissues in a multicellular organism.